{
  "gene_symbol": "MYRF",
  "term_id": "GO:0016540",
  "gene": "UniProtKB:Q9Y2G1",
  "term_label": "protein autoprocessing",
  "gene_name": "Myelin regulatory factor"
}